{
  "gene_name": "DNA-dependent protein kinase catalytic subunit",
  "gene_symbol": "PRKDC",
  "gene": "UniProtKB:P78527",
  "term_id": "GO:0004674",
  "term_label": "protein serine/threonine kinase activity"
}